{
  "term_id": "GO:0016064",
  "gene": "UniProtKB:P01772",
  "term_label": "immunoglobulin mediated immune response",
  "gene_symbol": "IGHV3-33",
  "gene_name": "Immunoglobulin heavy variable 3-33"
}